{
  "term_label": "ADP binding",
  "gene_name": "Phosphoglycerate kinase 1",
  "term_id": "GO:0043531",
  "gene": "UniProtKB:P00558",
  "gene_symbol": "PGK1"
}